{
  "term_id": "UNKNOWN:0002",
  "gene_symbol": "KANTR",
  "term_label": "Unknown biological process",
  "gene_name": "KANTR integral membrane protein",
  "gene": "UniProtKB:A0A1W2PQU2"
}